{
  "gene_symbol": "ITGA4",
  "term_id": "GO:0034668",
  "gene": "UniProtKB:P13612",
  "gene_name": "Integrin alpha-4",
  "term_label": "integrin alpha4-beta1 complex"
}